U6 snRNA 2'-O-ribose methyltransferase activity [GO:0180021] (molecular function) References: PMID:37403782 Sources: RHEA:63088 Relationships: is a type of small RNA 2'-O-methyltransferase activity [GO:0090486] Definition: Catalysis of the reaction: S-adenosyl-L-methionine + U6 snRNA = S-adenosyl-L-homocysteine + U6 containing a 3'-terminal 2'-O-methylnucleotide + H+.